{
  "gene_symbol": "LGALS3BP",
  "gene_name": "Galectin-3-binding protein",
  "term_id": "UNKNOWN:0002",
  "gene": "UniProtKB:Q08380",
  "term_label": "Unknown biological process"
}